mevalonate transport [GO:0015728] (biological process) Sources: GOC:krc Definition: The directed movement of mevalonate into, out of or within a cell, or between cells, by means of some agent such as a transporter or pore. Relationships: is a type of GO:0006810